cellular response to carcinoembryonic antigen [GO:1990831] (biological process) Relationships: is a type of cellular response to glycoprotein [GO:1904588] Also known as: cellular response to pregnancy specific glycoprotein Definition: Any process that results in a change in state or activity of a cell (in terms of movement, secretion, enzyme production, gene expression, etc.) as a result of a carcinoembryonic antigen stimulus. The carcinoembryonic antigens represent a family of glycoproteins. References: PMID:10202129, PMID:14597422